{
  "term_id": "GO:0005737",
  "term_label": "cytoplasm",
  "gene": "UniProtKB:P27361",
  "gene_symbol": "MAPK3",
  "gene_name": "Mitogen-activated protein kinase 3"
}